{
  "term_id": "GO:0008574",
  "term_label": "plus-end-directed microtubule motor activity",
  "gene_symbol": "KIF18B",
  "gene": "UniProtKB:Q86Y91",
  "gene_name": "Kinesin-like protein KIF18B"
}